{
  "gene_name": "Sodium-dependent neutral amino acid transporter SLC6A17",
  "term_id": "GO:0008021",
  "term_label": "synaptic vesicle",
  "gene_symbol": "SLC6A17",
  "gene": "UniProtKB:Q9H1V8"
}